{
  "gene_symbol": "POU4F1",
  "gene_name": "POU domain, class 4, transcription factor 1",
  "gene": "UniProtKB:Q01851",
  "term_id": "GO:0000981",
  "term_label": "DNA-binding transcription factor activity, RNA polymerase II-specific"
}